{
  "gene": "UniProtKB:A8MYZ5",
  "gene_name": "IQ domain-containing protein F6",
  "gene_symbol": "IQCF6",
  "term_label": "calmodulin binding",
  "term_id": "GO:0005516"
}